detection of nutrient [GO:0009594] (biological process) Definition: The series of events in which a nutrient stimulus is received by a cell and converted into a molecular signal. Sources: GOC:jl Also known as: detection of nutrients, nutrient sensing, perception of nutrients Relationships: is a type of GO:0007584; is a type of detection of chemical stimulus [GO:0009593] Subtypes: detection of folic acid [GO:0031318]